{
  "gene_name": "Hepcidin",
  "term_id": "UNKNOWN:0001",
  "gene": "UniProtKB:P81172",
  "gene_symbol": "HAMP",
  "term_label": "Unknown molecular function"
}